{
  "gene_name": "Tumor necrosis factor receptor superfamily member 6B",
  "term_id": "UNKNOWN:0002",
  "term_label": "Unknown biological process",
  "gene": "UniProtKB:O95407",
  "gene_symbol": "TNFRSF6B"
}